regulation of membrane potential in photoreceptor cell [GO:0016057] (BP) Subtypes: maintenance of membrane potential in photoreceptor cell by rhodopsin mediated signaling [GO:0016058] Relationships: is a type of GO:0042391 Sources: GOC:dph, GOC:hb, GOC:tb Also known as: changes in polarization state of photoreceptor cell membrane Definition: Hyperpolarization (vertebrates) or depolarization (invertebrates) of the photoreceptor cell membrane via closing/opening of cation specific channels as a result of signals generated by rhodopsin activation by a photon.